{
  "term_label": "Unknown cellular component",
  "term_id": "UNKNOWN:0003",
  "gene_name": "Uncharacterized protein C10orf143",
  "gene_symbol": "C10orf143",
  "gene": "UniProtKB:A0A1B0GUT2"
}